positive regulation of natural killer cell proliferation [GO:0032819] (biological process) Also known as: positive regulation of NK cell proliferation, up regulation of natural killer cell proliferation, up-regulation of natural killer cell proliferation, upregulation of natural killer cell proliferation, activation of natural killer cell proliferation, stimulation of natural killer cell proliferation Relationships: is_a positive regulation of natural killer cell activation [GO:0032816]; is a type of regulation of natural killer cell proliferation [GO:0032817]; is a type of positive regulation of lymphocyte proliferation [GO:0050671]; positively regulates natural killer cell proliferation [GO:0001787] Definition: Any process that activates or increases the frequency, rate or extent of natural killer cell proliferation. Subtypes: positive regulation of natural killer cell proliferation involved in immune response [GO:0032822] Sources: GOC:mah